{
  "gene_symbol": "CXorf51B",
  "term_label": "Unknown cellular component",
  "term_id": "UNKNOWN:0003",
  "gene": "UniProtKB:P0DPH9",
  "gene_name": "Uncharacterized protein CXorf51B"
}